{
  "term_id": "GO:0016791",
  "gene_name": "Pyridoxal phosphate phosphatase PHOSPHO2",
  "term_label": "phosphatase activity",
  "gene": "UniProtKB:Q8TCD6",
  "gene_symbol": "PHOSPHO2"
}